5-alpha-androstane-3-beta,17-beta-diol dehydrogenase (NADP+) activity [GO:0047024] (molecular function) Sources: RHEA:16297 Definition: Catalysis of the reaction: 5-alpha-androstane-3-beta,17-beta-diol + NADP+ = 17-beta-hydroxy-5-alpha-androstan-3-one + H+ + NADPH. Relationships: is a type of steroid dehydrogenase activity, acting on the CH-OH group of donors, NAD or NADP as acceptor [GO:0033764] Also known as: 3-beta(or 20-alpha)-hydroxysteroid dehydrogenase activity, 3beta(or 20alpha)-hydroxysteroid dehydrogenase activity, 3beta(or 20alpha)-hydroxysteroid:NADP+ oxidoreductase activity, 3beta,20alpha-hydroxysteroid oxidoreductase activity, dehydrogenase, 3beta,20alpha-hydroxy steroid, 5alpha-androstane-3beta,17beta-diol dehydrogenase activity, 3-beta-HSD activity, progesterone reductase activity